{
  "gene_name": "Probable sodium-coupled neutral amino acid transporter 6",
  "term_id": "GO:0005886",
  "gene_symbol": "SLC38A6",
  "gene": "UniProtKB:Q8IZM9",
  "term_label": "plasma membrane"
}